{
  "term_id": "GO:0032991",
  "gene": "UniProtKB:Q9H867",
  "gene_name": "Protein N-lysine methyltransferase METTL21D",
  "term_label": "protein-containing complex",
  "gene_symbol": "VCPKMT"
}